{
  "term_label": "spermatogenesis",
  "gene_name": "Testicular spindle-associated protein SHCBP1L",
  "gene_symbol": "SHCBP1L",
  "gene": "UniProtKB:Q9BZQ2",
  "term_id": "GO:0007283"
}